{
  "gene_name": "C2 domain-containing protein 3",
  "gene_symbol": "C2CD3",
  "gene": "UniProtKB:Q4AC94",
  "term_id": "GO:0005815",
  "term_label": "microtubule organizing center"
}